{
  "gene_name": "Homeobox protein Nkx-6.2",
  "gene_symbol": "NKX6-2",
  "gene": "UniProtKB:Q9C056",
  "term_label": "RNA polymerase II cis-regulatory region sequence-specific DNA binding",
  "term_id": "GO:0000978"
}